{
  "gene_symbol": "TMCC2",
  "term_id": "GO:0042982",
  "gene_name": "Transmembrane and coiled-coil domains protein 2",
  "gene": "UniProtKB:O75069",
  "term_label": "amyloid precursor protein metabolic process"
}